alpha,alpha-trehalose phosphorylase (configuration-retaining) activity [GO:0033832] (molecular function) Also known as: trehalose phosphorylase activity, alpha,alpha-trehalose:phosphate alpha-D-glucosyltransferase activity Relationships: is a type of glucosyltransferase activity [GO:0046527] Definition: Catalysis of the reaction: alpha,alpha-trehalose + phosphate = alpha-D-glucose + alpha-D-glucose 1-phosphate. Sources: RHEA:16257